{
  "gene": "UniProtKB:Q99873",
  "term_id": "GO:0006355",
  "term_label": "regulation of DNA-templated transcription",
  "gene_symbol": "PRMT1",
  "gene_name": "Protein arginine N-methyltransferase 1"
}